{
  "gene_name": "Solute carrier family 2, facilitated glucose transporter member 9",
  "gene": "UniProtKB:Q9NRM0",
  "term_id": "GO:0005886",
  "gene_symbol": "SLC2A9",
  "term_label": "plasma membrane"
}